{
  "gene_name": "Sperm mitochondrial-associated cysteine-rich protein",
  "gene_symbol": "SMCP",
  "term_label": "Unknown cellular component",
  "term_id": "UNKNOWN:0003",
  "gene": "UniProtKB:P49901"
}